{
  "term_label": "natural killer cell activation involved in immune response",
  "gene_symbol": "IFNA14",
  "gene": "UniProtKB:P01570",
  "term_id": "GO:0002323",
  "gene_name": "Interferon alpha-14"
}